{
  "gene_symbol": "TPO",
  "gene": "UniProtKB:P07202",
  "term_id": "GO:0004601",
  "term_label": "peroxidase activity",
  "gene_name": "Thyroid peroxidase"
}